{
  "gene_name": "Potassium voltage-gated channel subfamily G member 4",
  "term_id": "GO:0016020",
  "gene_symbol": "KCNG4",
  "gene": "UniProtKB:Q8TDN1",
  "term_label": "membrane"
}